{
  "term_id": "GO:0005615",
  "gene": "UniProtKB:Q8IU54",
  "gene_name": "Interferon lambda-1",
  "gene_symbol": "IFNL1",
  "term_label": "extracellular space"
}